{
  "gene_name": "Alpha-1D adrenergic receptor",
  "term_label": "cell-cell signaling",
  "gene": "UniProtKB:P25100",
  "term_id": "GO:0007267",
  "gene_symbol": "ADRA1D"
}